{
  "gene_symbol": "KHNYN",
  "gene_name": "Protein KHNYN",
  "term_id": "GO:0005634",
  "term_label": "nucleus",
  "gene": "UniProtKB:O15037"
}